X chromosome located dosage compensation complex, transcription activating [GO:0016456] (cellular component) Definition: An RNA-protein complex localized to the X chromosome of males where it is required for the hyper-transcriptional activation of the X chromosome. An example of this is found in Drosophila melanogaster. References: PMID:20622855 Sources: GOC:ma, GOC:mr, GOC:mtg_sensu, Wikipedia:XY_sex-determination_system Also known as: dosage compensation complex Relationships: is a type of dosage compensation complex [GO:0046536]; is a type of ribonucleoprotein complex [GO:1990904]; is part of GO:0000805